{
  "term_label": "Unknown molecular function",
  "gene": "UniProtKB:Q7Z2X7",
  "gene_symbol": "PAGE2",
  "term_id": "UNKNOWN:0001",
  "gene_name": "P antigen family member 2"
}